{
  "gene_name": "Fanconi anemia group C protein",
  "gene": "UniProtKB:Q00597",
  "term_label": "Unknown molecular function",
  "term_id": "UNKNOWN:0001",
  "gene_symbol": "FANCC"
}